{
  "gene": "UniProtKB:Q8TAU0",
  "gene_symbol": "NKX2-3",
  "gene_name": "Homeobox protein Nkx-2.3",
  "term_label": "RNA polymerase II cis-regulatory region sequence-specific DNA binding",
  "term_id": "GO:0000978"
}